{
  "gene_name": "Putative transcriptional regulator encoded by LINC00473",
  "gene": "UniProtKB:A8K010",
  "term_label": "Unknown biological process",
  "gene_symbol": "LINC00473",
  "term_id": "UNKNOWN:0002"
}